{
  "gene_name": "Forkhead box protein P2",
  "gene": "UniProtKB:O15409",
  "gene_symbol": "FOXP2",
  "term_label": "RNA polymerase II cis-regulatory region sequence-specific DNA binding",
  "term_id": "GO:0000978"
}